{
  "gene": "UniProtKB:Q5TGY1",
  "term_id": "UNKNOWN:0001",
  "gene_symbol": "TMCO4",
  "gene_name": "Transmembrane and coiled-coil domain-containing protein 4",
  "term_label": "Unknown molecular function"
}